{
  "gene": "UniProtKB:Q96RC9",
  "gene_name": "Olfactory receptor 8B4",
  "term_id": "GO:0007186",
  "term_label": "G protein-coupled receptor signaling pathway",
  "gene_symbol": "OR8B4"
}